{
  "term_label": "DNA-binding transcription factor activity, RNA polymerase II-specific",
  "gene_name": "Zinc finger protein 852",
  "gene_symbol": "ZNF852",
  "gene": "UniProtKB:Q6ZMS4",
  "term_id": "GO:0000981"
}